{
  "gene_name": "Interferon beta",
  "term_label": "extracellular space",
  "gene": "UniProtKB:P01574",
  "gene_symbol": "IFNB1",
  "term_id": "GO:0005615"
}